coniferyl-alcohol dehydrogenase activity [GO:0050268] (molecular function) Definition: Catalysis of the reaction: coniferyl alcohol + NADP+ = coniferyl aldehyde + NADPH. Also known as: coniferyl-alcohol:NADP+ oxidoreductase activity Relationships: is a type of GO:0016616 Sources: RHEA:22444